{
  "gene_name": "Solute carrier family 15 member 4",
  "term_id": "GO:0140206",
  "gene_symbol": "SLC15A4",
  "term_label": "dipeptide import across plasma membrane",
  "gene": "UniProtKB:Q8N697"
}